{
  "term_id": "GO:0005829",
  "term_label": "cytosol",
  "gene_symbol": "PDXP",
  "gene_name": "Chronophin",
  "gene": "UniProtKB:Q96GD0"
}